regulation of intracellular transport of viral material [GO:1901252] (biological process) Sources: GOC:TermGenie, GOC:bf, GOC:jl Relationships: is a type of regulation of biological process involved in symbiotic interaction [GO:0043903]; is a type of regulation of viral life cycle [GO:1903900]; regulates intracellular transport of virus [GO:0075733] Definition: Any process that modulates the frequency, rate or extent of egress of virus within host cell. Subtypes: negative regulation of intracellular transport of viral material [GO:1901253], positive regulation of intracellular transport of viral material [GO:1901254] Also known as: regulation of movement of virus within host cell, regulation of viral egress, regulation of egress of virus within host cell